{
  "gene_name": "Leucine-rich repeat and IQ domain-containing protein 4",
  "term_label": "Unknown molecular function",
  "gene": "UniProtKB:A6NIV6",
  "term_id": "UNKNOWN:0001",
  "gene_symbol": "LRRIQ4"
}